{
  "term_label": "M band",
  "gene": "UniProtKB:Q13203",
  "gene_symbol": "MYBPH",
  "term_id": "GO:0031430",
  "gene_name": "Myosin-binding protein H"
}